{
  "gene_symbol": "MDFIC",
  "term_label": "Unknown molecular function",
  "gene": "UniProtKB:Q9P1T7",
  "gene_name": "MyoD family inhibitor domain-containing protein",
  "term_id": "UNKNOWN:0001"
}